{
  "gene": "UniProtKB:P12272",
  "term_id": "GO:0007189",
  "term_label": "adenylate cyclase-activating G protein-coupled receptor signaling pathway",
  "gene_name": "Parathyroid hormone-related protein",
  "gene_symbol": "PTHLH"
}